{
  "term_id": "GO:0051607",
  "gene_symbol": "AICDA",
  "term_label": "defense response to virus",
  "gene_name": "Single-stranded DNA cytosine deaminase",
  "gene": "UniProtKB:Q9GZX7"
}